{
  "gene_symbol": "ABCD3",
  "term_id": "GO:0005324",
  "gene_name": "ATP-binding cassette sub-family D member 3",
  "term_label": "long-chain fatty acid transmembrane transporter activity",
  "gene": "UniProtKB:P28288"
}